{
  "gene": "UniProtKB:P63279",
  "gene_name": "SUMO-conjugating enzyme UBC9",
  "gene_symbol": "UBE2I",
  "term_label": "nucleus",
  "term_id": "GO:0005634"
}